{
  "gene_name": "Zinc finger protein 143",
  "term_label": "regulation of DNA-templated transcription",
  "gene_symbol": "ZNF143",
  "term_id": "GO:0006355",
  "gene": "UniProtKB:P52747"
}